{
  "gene_name": "PILR alpha-associated neural protein",
  "term_id": "UNKNOWN:0002",
  "gene_symbol": "PIANP",
  "gene": "UniProtKB:Q8IYJ0",
  "term_label": "Unknown biological process"
}